{
  "gene": "UniProtKB:Q9ULZ2",
  "term_id": "GO:0019901",
  "gene_symbol": "STAP1",
  "gene_name": "Signal-transducing adaptor protein 1",
  "term_label": "protein kinase binding"
}